{
  "gene_name": "mRNA-decapping enzyme 1B",
  "term_id": "GO:0031087",
  "term_label": "deadenylation-independent decapping of nuclear-transcribed mRNA",
  "gene": "UniProtKB:Q8IZD4",
  "gene_symbol": "DCP1B"
}